{
  "gene": "UniProtKB:Q3SY00",
  "term_id": "UNKNOWN:0001",
  "gene_name": "Testis-specific protein 10-interacting protein",
  "gene_symbol": "TSGA10IP",
  "term_label": "Unknown molecular function"
}